{
  "term_id": "GO:0051082",
  "gene_name": "UDP-glucose:glycoprotein glucosyltransferase 1",
  "gene_symbol": "UGGT1",
  "gene": "UniProtKB:Q9NYU2",
  "term_label": "unfolded protein binding"
}